negative regulation of protein import [GO:1904590] (biological process) References: PMID:11406629 Sources: GOC:TermGenie, GO_REF:0000058 Relationships: is a type of negative regulation of protein transport [GO:0051224]; is a type of GO:1904589; negatively regulates GO:0017038 Definition: Any process that stops, prevents or reduces the frequency, rate or extent of protein import. Also known as: down regulation of protein import, down regulation of protein uptake, down-regulation of protein import, down-regulation of protein uptake, downregulation of protein import, downregulation of protein uptake, negative regulation of protein uptake, inhibition of protein import, inhibition of protein uptake